phragmoplast microtubule organization [GO:0080175] (BP) Also known as: phragmoplast microtubule cytoskeleton organization, phragmoplast microtubule organisation Relationships: is a type of microtubule cytoskeleton organization [GO:0000226]; occurs in phragmoplast [GO:0009524] Definition: A process that is carried out at the cellular level which results in the assembly, arrangement of constituent parts, or disassembly of structures formed of microtubules and associated proteins in phragmoplast, a plant cell specific structure that forms during late cytokinesis. Phragmoplast serves as a scaffold for cell plate assembly and subsequent formation of a new cell wall separating the two daughter cells. References: PMID:19383896 Regulation: regulated by regulation of phragmoplast microtubule organization [GO:2000694]